{
  "term_label": "extracellular matrix assembly",
  "gene_symbol": "HAS3",
  "gene": "UniProtKB:O00219",
  "gene_name": "Hyaluronan synthase 3",
  "term_id": "GO:0085029"
}